{
  "term_label": "ubiquitin protein ligase activity",
  "gene_name": "E3 ubiquitin-protein ligase TRIM37",
  "term_id": "GO:0061630",
  "gene": "UniProtKB:O94972",
  "gene_symbol": "TRIM37"
}